{
  "gene_symbol": "BFSP1",
  "gene": "UniProtKB:Q12934",
  "term_label": "structural constituent of eye lens",
  "term_id": "GO:0005212",
  "gene_name": "Filensin"
}